{
  "gene": "UniProtKB:Q8N0Y5",
  "gene_name": "Olfactory receptor 8I2",
  "gene_symbol": "OR8I2",
  "term_label": "sensory perception of smell",
  "term_id": "GO:0007608"
}